{
  "term_label": "Unknown molecular function",
  "term_id": "UNKNOWN:0001",
  "gene_symbol": "CCDC126",
  "gene_name": "Coiled-coil domain-containing protein 126",
  "gene": "UniProtKB:Q96EE4"
}